regulation of inhibitory G protein-coupled receptor phosphorylation [GO:1904323] (biological process) Relationships: is a type of GO:0001932; regulates inhibitory G protein-coupled receptor phosphorylation [GO:0002030] Also known as: regulation of inhibitory G-protein coupled receptor phosphorylation Definition: Any process that modulates the frequency, rate or extent of inhibitory G protein-coupled receptor phosphorylation. References: PMID:15937517 Sources: GOC:TermGenie, GO_REF:0000058 Subtypes: negative regulation of inhibitory G protein-coupled receptor phosphorylation [GO:1904324], GO:1904325